{
  "gene_symbol": "VPS26C",
  "gene": "UniProtKB:O14972",
  "gene_name": "Vacuolar protein sorting-associated protein 26C",
  "term_label": "endosome",
  "term_id": "GO:0005768"
}